{
  "term_id": "GO:0004674",
  "term_label": "protein serine/threonine kinase activity",
  "gene": "UniProtKB:Q05513",
  "gene_name": "Protein kinase C zeta type",
  "gene_symbol": "PRKCZ"
}